positive regulation of Hulle cell development [GO:0070810] (biological process) Relationships: is_a GO:0010720; is a type of regulation of Hulle cell development [GO:0070808]; is a type of positive regulation of reproductive process [GO:2000243]; positively regulates Hulle cell development [GO:0070792] Sources: GOC:mah Definition: Any process that activates or increases the frequency, rate or extent of Hulle cell development, a process that leads to the formation of Hulle cells. Hulle cells are specialized multinucleate cells that originate from a nest-like aggregation of hyphae during sexual development and serve as nurse cells to the developing cleistothecium, or fruiting body.